{
  "gene_symbol": "TRAPPC3",
  "term_label": "cytosol",
  "term_id": "GO:0005829",
  "gene": "UniProtKB:O43617",
  "gene_name": "Trafficking protein particle complex subunit 3"
}